serine-based site-specific recombinase activity [GO:0160053] (molecular function) Definition: Catalysis of the formation of new phosphodiester bonds between a pair of short, unique DNA target sequences; occurs through a phosphoseryl intermediate in which the target sequence is first cleaved by the nucleophilic attack by a serine in the active site. References: PMID:16756503, PMID:29316791 Relationships: is a type of site-specific recombinase activity [GO:0009009]